{
  "gene_symbol": "NDFIP2",
  "gene": "UniProtKB:Q9NV92",
  "gene_name": "NEDD4 family-interacting protein 2",
  "term_label": "perinuclear region of cytoplasm",
  "term_id": "GO:0048471"
}